{
  "term_label": "transmembrane transporter binding",
  "gene_symbol": "LRRC26",
  "term_id": "GO:0044325",
  "gene": "UniProtKB:Q2I0M4",
  "gene_name": "Leucine-rich repeat-containing protein 26"
}